{
  "gene": "UniProtKB:Q9BYJ0",
  "term_id": "GO:0007267",
  "gene_name": "Fibroblast growth factor-binding protein 2",
  "term_label": "cell-cell signaling",
  "gene_symbol": "FGFBP2"
}